acetylcholinesterase activity [GO:0003990] (molecular function) Sources: EC:3.1.1.7 Definition: Catalysis of the reaction: acetylcholine + H2O = choline + acetate. Also known as: AcCholE, acetyl.beta-methylcholinesterase activity, acetylcholine acetylhydrolase activity, acetylcholine hydrolase activity, acetylthiocholinesterase activity, choline esterase I activity, true cholinesterase activity Relationships: is a type of cholinesterase activity [GO:0004104]